{
  "gene_symbol": "MAP10",
  "term_label": "mitotic spindle midzone",
  "gene": "UniProtKB:Q9P2G4",
  "term_id": "GO:1990023",
  "gene_name": "Microtubule-associated protein 10"
}